{
  "term_label": "N-acyltransferase activity",
  "term_id": "GO:0016410",
  "gene_name": "Phospholipase A and acyltransferase 2",
  "gene": "UniProtKB:Q9NWW9",
  "gene_symbol": "PLAAT2"
}